{
  "gene_name": "UL16-binding protein 3",
  "gene": "UniProtKB:Q9BZM4",
  "gene_symbol": "ULBP3",
  "term_id": "GO:0001916",
  "term_label": "positive regulation of T cell mediated cytotoxicity"
}